{
  "gene": "UniProtKB:Q9BVX2",
  "gene_name": "Transmembrane protein 106C",
  "term_id": "UNKNOWN:0003",
  "gene_symbol": "TMEM106C",
  "term_label": "Unknown cellular component"
}